{
  "gene_symbol": "KCNQ2",
  "gene_name": "Potassium voltage-gated channel subfamily KQT member 2",
  "gene": "UniProtKB:O43526",
  "term_label": "voltage-gated potassium channel complex",
  "term_id": "GO:0008076"
}